{
  "gene_name": "Protein PML",
  "term_id": "GO:0016605",
  "gene_symbol": "PML",
  "term_label": "PML body",
  "gene": "UniProtKB:P29590"
}